L-propargylglycine biosynthetic process [GO:0062143] (biological process) References: PMID:30867596 Definition: The chemical reactions and pathways resulting in the formation of L-propargylglycine (Pra). L-propargylglycine is an antibiotic produced by Streptomyces bacteria. Relationships: is a type of GO:0170034; is a type of non-proteinogenic amino acid biosynthetic process [GO:0170043]